{
  "gene_symbol": "KCTD16",
  "term_id": "GO:0045211",
  "gene": "UniProtKB:Q68DU8",
  "term_label": "postsynaptic membrane",
  "gene_name": "BTB_POZ domain-containing protein KCTD16"
}